{
  "term_label": "Unknown molecular function",
  "gene_name": "Clusterin-associated protein 1",
  "gene": "UniProtKB:Q96AJ1",
  "term_id": "UNKNOWN:0001",
  "gene_symbol": "CLUAP1"
}